{
  "gene_symbol": "TRDJ1",
  "term_id": "UNKNOWN:0003",
  "gene": "UniProtKB:A0A075B706",
  "term_label": "Unknown cellular component",
  "gene_name": "T cell receptor delta joining 1"
}